regulation of protein catabolic process [GO:0042176] (biological process) Definition: Any process that modulates the frequency, rate or extent of the chemical reactions and pathways resulting in the breakdown of a protein by the destruction of the native, active configuration, with or without the hydrolysis of peptide bonds. Sources: GOC:go_curators, GOC:jl Also known as: regulation of cellular protein breakdown, regulation of cellular protein catabolic process, regulation of cellular protein catabolism, regulation of cellular protein degradation, regulation of protein breakdown, regulation of protein catabolism, regulation of protein degradation, regulation of cyclin breakdown, regulation of cyclin catabolic process, regulation of cyclin catabolism, regulation of cyclin degradation, regulation of degradation of cyclin Relationships: is_a regulation of catabolic process [GO:0009894]; is a type of regulation of protein metabolic process [GO:0051246]; regulates GO:0030163 Subtypes: regulation of PSII associated light-harvesting complex II catabolic process [GO:0010550], regulation of low-density lipoprotein particle receptor catabolic process [GO:0032803], negative regulation of protein catabolic process [GO:0042177], GO:0045732, regulation of membrane protein ectodomain proteolysis [GO:0051043], regulation of elastin catabolic process [GO:0060310], regulation of proteasomal protein catabolic process [GO:0061136], GO:0099575, regulation of protein catabolic process at postsynapse, modulating synaptic transmission [GO:0099576], GO:1904350, regulation of chaperone-mediated autophagy [GO:1904714]